{
  "gene_symbol": "TWIST2",
  "term_id": "GO:0000981",
  "gene": "UniProtKB:Q8WVJ9",
  "gene_name": "Twist-related protein 2",
  "term_label": "DNA-binding transcription factor activity, RNA polymerase II-specific"
}